4-(trimethylammonio)butanoate transport [GO:1900751] (biological process) References: PMID:16365044, PMID:20357772, PMID:20829798 Sources: GOC:TermGenie Relationships: is a type of organic cation transport [GO:0015695]; is_a amino-acid betaine transport [GO:0015838] Definition: The directed movement of a 4-(trimethylammonio)butanoate into, out of or within a cell, or between cells, by means of some agent such as a transporter or pore. Also known as: 4-(N-trimethylamino)butyrate transport, 4-butyrobetaine transport, gamma-Butyrobetain transport, gamma-butyrobetaine transport, Actinine transport, C7H15NO2 transport, butyrobetaine transport, deoxycarnitine transport